{
  "term_id": "GO:0034476",
  "gene_symbol": "EXOSC9",
  "gene": "UniProtKB:Q06265",
  "term_label": "U5 snRNA 3'-end processing",
  "gene_name": "Exosome complex component RRP45"
}